myosin II binding [GO:0045159] (molecular function) Relationships: is a type of myosin binding [GO:0017022] References: PMID:27697842 Sources: GOC:mah Subtypes: myosin II light chain binding [GO:0032033], GO:0032038 Definition: Binding to a class II myosin, any member of the class of 'conventional' double-headed myosins that includes muscle myosin.